{
  "term_id": "UNKNOWN:0002",
  "gene_symbol": "TMEM143",
  "gene_name": "Transmembrane protein 143",
  "gene": "UniProtKB:Q96AN5",
  "term_label": "Unknown biological process"
}